{
  "term_label": "Unknown molecular function",
  "gene_name": "Integrator complex subunit 2",
  "gene_symbol": "INTS2",
  "term_id": "UNKNOWN:0001",
  "gene": "UniProtKB:Q9H0H0"
}